{
  "gene_name": "Keratin, type I cuticular Ha5",
  "term_id": "GO:0002009",
  "term_label": "morphogenesis of an epithelium",
  "gene": "UniProtKB:Q92764",
  "gene_symbol": "KRT35"
}